negative regulation of tRNA catabolic process [GO:1902371] (biological process) Also known as: down regulation of tRNA breakdown, down regulation of tRNA catabolic process, down regulation of tRNA catabolism, down regulation of tRNA degradation, down-regulation of tRNA breakdown, down-regulation of tRNA catabolic process, down-regulation of tRNA catabolism, down-regulation of tRNA degradation, downregulation of tRNA breakdown, downregulation of tRNA catabolic process, downregulation of tRNA catabolism, downregulation of tRNA degradation, negative regulation of tRNA breakdown, negative regulation of tRNA catabolism, negative regulation of tRNA degradation, inhibition of tRNA breakdown, inhibition of tRNA catabolic process, inhibition of tRNA catabolism, inhibition of tRNA degradation Relationships: is a type of negative regulation of RNA catabolic process [GO:1902369]; is a type of GO:1902370; is_a negative regulation of tRNA metabolic process [GO:1903327]; negatively regulates tRNA decay [GO:0016078] Definition: Any process that stops, prevents or reduces the frequency, rate or extent of tRNA catabolic process. References: PMID:22919049 Sources: GOC:TermGenie, GOC:bf Subtypes: GO:0036416